{
  "gene_symbol": "SPATA4",
  "term_id": "GO:0008017",
  "gene": "UniProtKB:Q8NEY3",
  "term_label": "microtubule binding",
  "gene_name": "Spermatogenesis-associated protein 4"
}